theanine hydrolase activity [GO:0050330] (molecular function) Definition: Catalysis of the reaction: N(5)-ethyl-L-glutamine + H2O = L-glutamate + ethylamine. Sources: EC:3.5.1.65, RHEA:18013 Also known as: 5-N-ethyl-L-glutamine amidohydrolase activity, L-theanine amidohydrolase activity, N5-ethyl-L-glutamine amidohydrolase activity Relationships: is a type of hydrolase activity, acting on carbon-nitrogen (but not peptide) bonds, in linear amides [GO:0016811]